regulation of natural killer cell mediated immunity [GO:0002715] (biological process) Also known as: regulation of NK cell mediated immunity, regulation of natural killer cell activity Subtypes: negative regulation of natural killer cell mediated immunity [GO:0002716], positive regulation of natural killer cell mediated immunity [GO:0002717], GO:0002727, regulation of natural killer cell mediated immune response to tumor cell [GO:0002855], GO:0042269 Relationships: is a type of regulation of lymphocyte mediated immunity [GO:0002706]; is_a GO:0045088; RO_0002211 GO:0002228 Definition: Any process that modulates the frequency, rate, or extent of natural killer cell mediated immunity. Sources: GOC:add